{
  "gene_name": "Small G protein signaling modulator 2",
  "gene": "UniProtKB:O43147",
  "gene_symbol": "SGSM2",
  "term_label": "GTPase activator activity",
  "term_id": "GO:0005096"
}